negative regulation of muscle contraction [GO:0045932] (biological process) Relationships: is a type of regulation of muscle contraction [GO:0006937]; is a type of GO:0051241; negatively regulates muscle contraction [GO:0006936] Subtypes: negative regulation of smooth muscle contraction [GO:0045986], negative regulation of striated muscle contraction [GO:0045988], GO:1904113 Sources: GOC:go_curators Also known as: down regulation of muscle contraction, down-regulation of muscle contraction, downregulation of muscle contraction, inhibition of muscle contraction Definition: Any process that stops, prevents, or reduces the frequency, rate or extent of muscle contraction.